{
  "term_label": "Unknown biological process",
  "gene_name": "Dehydrogenase_reductase SDR family member 7",
  "gene_symbol": "DHRS7",
  "term_id": "UNKNOWN:0002",
  "gene": "UniProtKB:Q9Y394"
}